{
  "gene_symbol": "TMEM45B",
  "term_id": "UNKNOWN:0001",
  "gene_name": "Transmembrane protein 45B",
  "gene": "UniProtKB:Q96B21",
  "term_label": "Unknown molecular function"
}